{
  "gene": "UniProtKB:P43220",
  "term_label": "plasma membrane",
  "gene_name": "Glucagon-like peptide 1 receptor",
  "gene_symbol": "GLP1R",
  "term_id": "GO:0005886"
}